{
  "term_label": "regulation of cell migration",
  "term_id": "GO:0030334",
  "gene": "UniProtKB:O00230",
  "gene_symbol": "CORT",
  "gene_name": "Cortistatin"
}